mechanosensitive monoatomic cation channel activity [GO:0140135] (molecular function) Also known as: mechanosensitive cation channel activity, mechanically-gated cation channel activity Relationships: is a type of monoatomic cation channel activity [GO:0005261]; is a type of mechanosensitive monoatomic ion channel activity [GO:0008381] Subtypes: stretch-activated, monoatomic cation-selective, calcium channel activity [GO:0015275], mechanosensitive potassium channel activity [GO:0098782], mechanosensitive voltage-gated sodium channel activity [GO:0101013] References: PMID:22343900 Sources: GOC:ha Definition: Enables the transmembrane transfer of a monoatomic cation by a channel that opens in response to a mechanical stress.